{
  "term_label": "cellular response to amino acid starvation",
  "gene": "UniProtKB:Q13049",
  "term_id": "GO:0034198",
  "gene_symbol": "TRIM32",
  "gene_name": "E3 ubiquitin-protein ligase TRIM32"
}